{
  "gene_symbol": "HKDC1",
  "gene_name": "Hexokinase HKDC1",
  "term_label": "glycolytic process",
  "gene": "UniProtKB:Q2TB90",
  "term_id": "GO:0006096"
}